siRNA transcription [GO:0140745] (biological process) References: PMID:23001036 Relationships: is a type of RNA-templated transcription [GO:0001172] Definition: The transcription of a small interfering RNA from an RNA template.